{
  "gene_name": "Zinc transporter ZIP5",
  "term_id": "GO:0030003",
  "term_label": "intracellular monoatomic cation homeostasis",
  "gene": "UniProtKB:Q6ZMH5",
  "gene_symbol": "SLC39A5"
}